{
  "gene": "UniProtKB:Q9UK23",
  "gene_name": "N-acetylglucosamine-1-phosphodiester alpha-N-acetylglucosaminidase",
  "gene_symbol": "NAGPA",
  "term_label": "Unknown cellular component",
  "term_id": "UNKNOWN:0003"
}